musculoskeletal movement, spinal reflex action [GO:0050883] (biological process) Relationships: is a type of musculoskeletal movement [GO:0050881]; is a type of reflex [GO:0060004] Definition: Involuntary movement caused by the application of a stimulus to an organism and a subsequent movement. The signal processing of this movement takes place in the spinal cord. Sources: GOC:dph